{
  "gene": "UniProtKB:Q13285",
  "gene_name": "Steroidogenic factor 1",
  "gene_symbol": "NR5A1",
  "term_id": "GO:0090575",
  "term_label": "RNA polymerase II transcription regulator complex"
}